K48-linked polyubiquitin modification-dependent protein binding [GO:0036435] (molecular function) Definition: Binding to a protein upon poly-ubiquitination formed by linkages between lysine residues at position 48 in the target protein. Relationships: is a type of polyubiquitin modification-dependent protein binding [GO:0031593] References: PMID:20739285 Sources: GOC:al